{
  "term_id": "UNKNOWN:0003",
  "term_label": "Unknown cellular component",
  "gene_name": "Ganglioside-induced differentiation-associated protein 1-like 1",
  "gene": "UniProtKB:Q96MZ0",
  "gene_symbol": "GDAP1L1"
}